{
  "gene_name": "DNA polymerase epsilon subunit 3",
  "gene": "UniProtKB:Q9NRF9",
  "term_id": "GO:0006974",
  "term_label": "DNA damage response",
  "gene_symbol": "POLE3"
}